phenylacetaldoxime dehydratase activity [GO:0018814] (molecular function) Definition: Catalysis of the reaction: (trans)-phenylacetaldoxime = H2O + phenylacetonitrile. Also known as: (Z)-phenylacetaldehyde-oxime hydro-lyase activity, arylacetaldoxime dehydratase activity, PAOx dehydratase activity Relationships: is a type of nitrogen-oxygen lyase activity [GO:0141122] References: PMID:25015725 Sources: RHEA:20069